1-phosphatidylinositol 4-kinase activator activity [GO:0098744] (molecular function) References: PMID:21288895 Definition: Binds to and increases the activity of 1-phosphatidylinositol 4-kinase. Relationships: is a type of kinase activator activity [GO:0019209]; positively regulates GO:0004430